{
  "gene_name": "BTB_POZ domain-containing protein 7",
  "gene": "UniProtKB:Q9P203",
  "term_id": "UNKNOWN:0003",
  "gene_symbol": "BTBD7",
  "term_label": "Unknown cellular component"
}